{
  "gene": "UniProtKB:O15243",
  "gene_name": "Leptin receptor gene-related protein",
  "term_id": "UNKNOWN:0001",
  "gene_symbol": "LEPROT",
  "term_label": "Unknown molecular function"
}